{
  "gene_symbol": "FGA",
  "gene": "UniProtKB:P02671",
  "term_label": "platelet aggregation",
  "term_id": "GO:0070527",
  "gene_name": "Fibrinogen alpha chain"
}